positive regulation of natural killer cell tolerance induction [GO:0002873] (biological process) Sources: GOC:add Definition: Any process that activates or increases the frequency, rate, or extent of natural killer cell tolerance induction. Also known as: positive regulation of NK cell tolerance induction, up regulation of natural killer cell tolerance induction, up-regulation of natural killer cell tolerance induction, upregulation of natural killer cell tolerance induction, activation of natural killer cell tolerance induction, stimulation of natural killer cell tolerance induction Relationships: is a type of GO:0002645; is a type of regulation of acute inflammatory response [GO:0002673]; is a type of GO:0002871; positively regulates natural killer cell tolerance induction [GO:0002519]